formin-nucleated actin cable [GO:0070648] (cellular component) Definition: An actin filament bundle that consists of short filaments organized into bundles of uniform polarity, and is nucleated by formins. In fungal cells, myosin motors transport cargo along actin cables toward sites of polarized cell growth; actin cables may play a similar role in pollen tube growth. Relationships: is a type of parallel actin filament bundle [GO:0097518] References: PMID:14671023, PMID:16959963